{
  "term_label": "midbody",
  "gene_symbol": "ZFYVE19",
  "term_id": "GO:0030496",
  "gene": "UniProtKB:Q96K21",
  "gene_name": "Abscission_NoCut checkpoint regulator"
}